{
  "gene_symbol": "DCUN1D3",
  "gene": "UniProtKB:Q8IWE4",
  "gene_name": "DCN1-like protein 3",
  "term_label": "ubiquitin-like protein binding",
  "term_id": "GO:0032182"
}